{
  "gene": "UniProtKB:P35244",
  "gene_symbol": "RPA3",
  "gene_name": "Replication protein A 14 kDa subunit",
  "term_id": "GO:0006298",
  "term_label": "mismatch repair"
}